{
  "term_id": "UNKNOWN:0002",
  "gene_symbol": "EXTL1",
  "gene": "UniProtKB:Q92935",
  "gene_name": "Exostosin-like 1",
  "term_label": "Unknown biological process"
}